positive regulation of induction of conjugation with cellular fusion [GO:1900237] (biological process) Sources: GOC:TermGenie Also known as: up regulation of induction of conjugation with cellular fusion, up-regulation of induction of conjugation with cellular fusion, upregulation of induction of conjugation with cellular fusion Definition: Any process that activates or increases the frequency, rate or extent of induction of conjugation with cellular fusion. Relationships: is a type of positive regulation of conjugation with cellular fusion [GO:0031139]; positively regulates induction of conjugation with cellular fusion [GO:0010514]